neurotensin receptor activity, non-G protein-coupled [GO:0030379] (molecular function) Also known as: neurotensin receptor activity, non G protein coupled, neurotensin receptor activity, non-G-protein coupled, non G protein coupled neurotensin receptor activity, non-G-protein coupled neurotensin receptor activity, non-G-protein-coupled neurotensin receptor activity References: PMID:9756851 Sources: GOC:mah, GOC:signaling Relationships: is a type of transmembrane signaling receptor activity [GO:0004888] Definition: Combining with neurotensin, a neuropeptide active in the central and peripheral nervous system in mammals, and transmitting the signal from one side of the membrane to the other by a mechanism independent of coupling to G proteins.